lysine 6-dehydrogenase activity [GO:0050303] (molecular function) Also known as: L-lysine 6-dehydrogenase activity, L-lysine epsilon-dehydrogenase activity, L-lysine:NAD+ 6-oxidoreductase (deaminating), LysDH activity Definition: Catalysis of the reaction: H2O + NAD+ + L-lysine = NH3 + NADH + allysine. Relationships: is a type of oxidoreductase activity, acting on the CH-NH2 group of donors, NAD or NADP as acceptor [GO:0016639] Sources: EC:1.4.1.18, MetaCyc:LYSINE-6-DEHYDROGENASE-RXN, RHEA:12408 Note: Note that this term has a MetaCyc pathway reference as the pathway only has a single step.